1-deoxy-11-oxopentalenate oxygenase activity [GO:0102285] (molecular function) Sources: GOC:pz, RHEA:34635 Relationships: is a type of oxidoreductase activity, acting on paired donors, with incorporation or reduction of molecular oxygen, NAD(P)H as one donor, and incorporation of one atom of oxygen [GO:0016709] Definition: Catalysis of the reaction: 1-deoxy-11-oxopentalenate + O2 + NADPH + H+ = pentalenolactone D + H2O + NADP.